filamentous actin [GO:0031941] (cellular component) Definition: A two-stranded helical polymer of the protein actin. Also known as: F-actin Note: Note that this term refers only to the actin portion of a microfilament, and does not encompass associated proteins. See also the cellular component term 'actin filament ; GO:0005884'. Sources: GOC:mah Relationships: is a type of protein-containing complex [GO:0032991]; is part of actin filament [GO:0005884]